{
  "gene_name": "Thrombospondin type-1 domain-containing protein 1",
  "gene": "UniProtKB:Q9NS62",
  "term_label": "Unknown molecular function",
  "gene_symbol": "THSD1",
  "term_id": "UNKNOWN:0001"
}